interleukin-1 beta production [GO:0032611] (biological process) Definition: The appearance of interleukin-1 beta due to biosynthesis or secretion following a cellular stimulus, resulting in an increase in its intracellular or extracellular levels. Relationships: is a type of interleukin-1 production [GO:0032612] Also known as: IL-1 beta production, interleukin-1 beta biosynthetic process, interleukin-1 beta secretion Regulation: regulated by regulation of interleukin-1 beta production [GO:0032651]; negatively regulated by negative regulation of interleukin-1 beta production [GO:0032691]; positively regulated by positive regulation of interleukin-1 beta production [GO:0032731] Sources: GOC:mah